regulation of phosphate transport [GO:0010966] (biological process) Definition: Any process that modulates the frequency, rate or extent of phosphate transport. Phosphate transport is the directed movement of phosphate into, out of or within a cell, or between cells, by means of some agent such as a transporter or pore. Relationships: is a type of regulation of transport [GO:0051049]; regulates phosphate ion transport [GO:0006817] Sources: GOC:dph, GOC:tb Subtypes: regulation of sodium-dependent phosphate transport [GO:2000118], regulation of phosphate transmembrane transport [GO:2000185]